{
  "gene": "UniProtKB:P55211",
  "term_id": "GO:0043525",
  "gene_symbol": "CASP9",
  "gene_name": "Caspase-9",
  "term_label": "positive regulation of neuron apoptotic process"
}